negative regulation of glutamatergic neuron differentiation [GO:0120007] (biological process) Definition: Any process that stops, prevents or reduces the frequency, rate or extent of glutamatergic neuron differentiation. References: PMID:24030726 Relationships: is a type of negative regulation of neuron differentiation [GO:0045665]; is a type of regulation of glutamatergic neuron differentiation [GO:0120006]; negatively regulates glutamatergic neuron differentiation [GO:1905962]